{
  "term_label": "cellular response to glucocorticoid stimulus",
  "gene": "UniProtKB:Q9HAW7",
  "gene_symbol": "UGT1A7",
  "term_id": "GO:0071385",
  "gene_name": "UDP-glucuronosyltransferase 1A7"
}